{
  "gene": "UniProtKB:Q8NGS5",
  "gene_symbol": "OR13C4",
  "gene_name": "Olfactory receptor 13C4",
  "term_id": "GO:0004984",
  "term_label": "olfactory receptor activity"
}